{
  "term_id": "GO:0043204",
  "gene_name": "High affinity choline transporter 1",
  "term_label": "perikaryon",
  "gene": "UniProtKB:Q9GZV3",
  "gene_symbol": "SLC5A7"
}